{
  "term_label": "cell surface receptor signaling pathway via JAK-STAT",
  "gene": "UniProtKB:Q9UBD9",
  "gene_name": "Cardiotrophin-like cytokine factor 1",
  "gene_symbol": "CLCF1",
  "term_id": "GO:0007259"
}